has_obo_namespace [oboInOwl#hasOBONamespace]